positive regulation of signaling [GO:0023056] (biological process) Also known as: positive regulation of signalling process, positive regulation of signaling process Sources: GOC:mtg_signal Definition: Any process that activates, maintains or increases the frequency, rate or extent of a signaling process. Subtypes: positive regulation of receptor recycling [GO:0001921], positive regulation of signal transduction [GO:0009967], positive regulation of hormone secretion [GO:0046887], positive regulation of synaptic transmission [GO:0050806], positive regulation of Wnt protein secretion [GO:0061357], positive regulation of c-di-GMP signaling [GO:0061941], GO:1900144, GO:1905434 Relationships: is a type of regulation of signaling [GO:0023051]; is a type of positive regulation of biological process [GO:0048518]; RO_0002213 GO:0023052